haloalkane dehalogenase activity [GO:0018786] (molecular function) Relationships: is a type of hydrolase activity, acting on acid halide bonds, in C-halide compounds [GO:0019120] Definition: Catalysis of the reaction: 1-haloalkane + H2O = a primary alcohol + halide. Also known as: 1-chlorohexane halidohydrolase activity, 1-haloalkane dehalogenase activity, 1-haloalkane halidohydrolase activity References: PMID:3624201 Sources: RHEA:19081